{
  "term_label": "nucleolus",
  "gene_name": "Nuclear nucleic acid-binding protein C1D",
  "gene_symbol": "C1D",
  "gene": "UniProtKB:Q13901",
  "term_id": "GO:0005730"
}